{
  "term_label": "negative regulation of cell adhesion",
  "term_id": "GO:0007162",
  "gene": "UniProtKB:O15031",
  "gene_name": "Plexin-B2",
  "gene_symbol": "PLXNB2"
}